(+)-pinoresinol biosynthetic process [GO:1902126] (biological process) References: PMID:8910615, PMID:9872995 Sources: GOC:TermGenie Also known as: (+)-pinoresinol anabolism, (+)-pinoresinol biosynthesis, (+)-pinoresinol formation, (+)-pinoresinol synthesis Definition: The chemical reactions and pathways resulting in the formation of (+)-pinoresinol. Relationships: is a type of lignan biosynthetic process [GO:0009807]; is a type of benzene-containing compound metabolic process [GO:0042537]; is a type of phenol-containing compound biosynthetic process [GO:0046189]; is_a ether biosynthetic process [GO:1901503]